{
  "gene_name": "RNA-binding motif protein, Y chromosome, family 1 member B",
  "term_label": "mRNA splicing, via spliceosome",
  "gene": "UniProtKB:A6NDE4",
  "term_id": "GO:0000398",
  "gene_symbol": "RBMY1B"
}